{
  "term_label": "plasma membrane",
  "term_id": "GO:0005886",
  "gene_symbol": "IRS1",
  "gene": "UniProtKB:P35568",
  "gene_name": "Insulin receptor substrate 1"
}